positive regulation of protein autoubiquitination [GO:1902499] (biological process) References: PMID:24069405 Sources: GOC:TermGenie, GOC:rb Also known as: positive regulation of protein auto-ubiquitination, positive regulation of protein auto-ubiquitinylation, positive regulation of protein autoubiquitinylation, positive regulation of protein self-ubiquitination, positive regulation of protein self-ubiquitinylation, up regulation of protein auto-ubiquitination, up regulation of protein auto-ubiquitinylation, up regulation of protein autoubiquitination, up regulation of protein autoubiquitinylation, up regulation of protein self-ubiquitination, up regulation of protein self-ubiquitinylation, up-regulation of protein auto-ubiquitination, up-regulation of protein auto-ubiquitinylation, up-regulation of protein autoubiquitination, up-regulation of protein autoubiquitinylation, up-regulation of protein self-ubiquitination, up-regulation of protein self-ubiquitinylation, upregulation of protein auto-ubiquitination, upregulation of protein auto-ubiquitinylation, upregulation of protein autoubiquitination, upregulation of protein autoubiquitinylation, upregulation of protein self-ubiquitination, upregulation of protein self-ubiquitinylation, activation of protein auto-ubiquitination, activation of protein auto-ubiquitinylation, activation of protein autoubiquitination, activation of protein autoubiquitinylation, activation of protein self-ubiquitination, activation of protein self-ubiquitinylation Relationships: is a type of positive regulation of protein ubiquitination [GO:0031398]; is a type of regulation of protein autoubiquitination [GO:1902498]; positively regulates protein autoubiquitination [GO:0051865] Definition: Any process that activates or increases the frequency, rate or extent of protein autoubiquitination.